{
  "term_label": "transcription coactivator activity",
  "gene_symbol": "SS18L1",
  "term_id": "GO:0003713",
  "gene": "UniProtKB:O75177",
  "gene_name": "Calcium-responsive transactivator"
}